{
  "term_label": "sodium channel regulator activity",
  "term_id": "GO:0017080",
  "gene_symbol": "FXYD3",
  "gene_name": "FXYD domain-containing ion transport regulator 3",
  "gene": "UniProtKB:Q14802"
}